germ tube septin cap [GO:0032171] (cellular component) References: PMID:16151244 Sources: GOC:krc Relationships: is_a septin cap [GO:0032159]; is part of GO:0032179 Definition: A faint structure formed of septins found at the leading edge of growth in germ tubes of fungal cells growing filamentously. This cap of septins colocalizes with a region of the plasma membrane that is rich in ergosterol.